MCM8-MCM9 complex [GO:0097362] (cellular component) Relationships: is a type of MCM complex [GO:0042555] Definition: A hexameric protein complex composed of MCM8 and MCM9 and involved in homologous recombination repair following DNA interstrand cross-links. References: PMID:22771115, PMID:22771120 Sources: GOC:sp